serine O-acyltransferase activity [GO:0016412] (molecular function) Sources: RHEA:68272 Subtypes: serine O-acetyltransferase activity [GO:0009001] Definition: Catalysis of the reaction: a fatty acyl-CoA + L-seryl-[protein] = CoA + O-fatty acyl-L-seryl-[protein]. Relationships: is_a O-acyltransferase activity [GO:0008374]